{
  "gene_symbol": "SLC25A35",
  "term_label": "Unknown cellular component",
  "gene": "UniProtKB:Q3KQZ1",
  "term_id": "UNKNOWN:0003",
  "gene_name": "Solute carrier family 25 member 35"
}